triplet codon-amino acid adaptor activity [GO:0030533] (molecular function) Definition: The codon binding activity of a tRNA that positions an activated amino acid, mediating its insertion at the correct point in the sequence of a nascent polypeptide chain during protein synthesis. Note: Note that this term can be used in place of the obsolete term 'transfer RNA ; GO:0005563'. Subtypes: UUU codon-amino acid adaptor activity [GO:0033401], UUC codon-amino acid adaptor activity [GO:0033402], UUA codon-amino acid adaptor activity [GO:0033403], GO:0033404, UCU codon-amino acid adaptor activity [GO:0033405], UCC codon-amino acid adaptor activity [GO:0033406], GO:0033407, UCG codon-amino acid adaptor activity [GO:0033408], UAU codon-amino acid adaptor activity [GO:0033409], UAC codon-amino acid adaptor activity [GO:0033410], UAA codon-amino acid adaptor activity [GO:0033411], UAG codon-amino acid adaptor activity [GO:0033412], UGU codon-amino acid adaptor activity [GO:0033413], UGC codon-amino acid adaptor activity [GO:0033414], UGA codon-amino acid adaptor activity [GO:0033415], UGG codon-amino acid adaptor activity [GO:0033416], CUU codon-amino acid adaptor activity [GO:0033417], CUC codon-amino acid adaptor activity [GO:0033418], CUA codon-amino acid adaptor activity [GO:0033419], CUG codon-amino acid adaptor activity [GO:0033420], CCU codon-amino acid adaptor activity [GO:0033421], CCC codon-amino acid adaptor activity [GO:0033422], CCA codon-amino acid adaptor activity [GO:0033423], CCG codon-amino acid adaptor activity [GO:0033424], GO:0033425, CAC codon-amino acid adaptor activity [GO:0033426], GO:0033427, CAG codon-amino acid adaptor activity [GO:0033428], GO:0033429, CGC codon-amino acid adaptor activity [GO:0033430], GO:0033431, CGG codon-amino acid adaptor activity [GO:0033432], AUU codon-amino acid adaptor activity [GO:0033433], AUC codon-amino acid adaptor activity [GO:0033434], GO:0033435, AUG codon-amino acid adaptor activity [GO:0033436], ACU codon-amino acid adaptor activity [GO:0033437], GO:0033438, GO:0033439, GO:0033440, AAU codon-amino acid adaptor activity [GO:0033441], AAC codon-amino acid adaptor activity [GO:0033442], GO:0033443, AAG codon-amino acid adaptor activity [GO:0033444], GO:0033445, AGC codon-amino acid adaptor activity [GO:0033446], AGA codon-amino acid adaptor activity [GO:0033447], AGG codon-amino acid adaptor activity [GO:0033448], GUU codon-amino acid adaptor activity [GO:0033449], GO:0033450, GUA codon-amino acid adaptor activity [GO:0033451], GUG codon-amino acid adaptor activity [GO:0033452], GO:0033453, GO:0033454, GCA codon-amino acid adaptor activity [GO:0033455], GCG codon-amino acid adaptor activity [GO:0033456], GAU codon-amino acid adaptor activity [GO:0033457], GAC codon-amino acid adaptor activity [GO:0033458], GAA codon-amino acid adaptor activity [GO:0033459], GO:0033460, GGU codon-amino acid adaptor activity [GO:0033461], GGC codon-amino acid adaptor activity [GO:0033462], GGA codon-amino acid adaptor activity [GO:0033463], GGG codon-amino acid adaptor activity [GO:0033464] Also known as: tRNA, transfer RNA Relationships: is a type of mRNA binding [GO:0003729]; is a type of molecular adaptor activity [GO:0060090]; is part of translation [GO:0006412] Sources: GOC:hjd, GOC:mtg_MIT_16mar07, ISBN:0198506732